{
  "gene_symbol": "PRDM15",
  "term_id": "GO:0005634",
  "gene": "UniProtKB:P57071",
  "term_label": "nucleus",
  "gene_name": "PR domain zinc finger protein 15"
}